omega speckle [GO:0035062] (cellular component) Definition: A nucleoplasmic speckle distributed in the interchromatin space of cells in close proximity to chromatin. Omega speckles are distinct from interchromatin granules and contain heterogeneous nuclear RNA-binding proteins (hnRNPs). Relationships: is a type of nuclear speck [GO:0016607] References: PMID:10984439 Sources: GOC:bf